eriodictyol 4'-O-methyltransferase activity [GO:0102762] (molecular function) Sources: GOC:pz, MetaCyc:RXN-7754 Relationships: is a type of GO:0008168 Definition: Catalysis of the reaction: eriodictyol + S-adenosyl-L-methionine = H+ + hesperetin(1-) + S-adenosyl-L-homocysteine.